positive regulation of mammary gland epithelial cell proliferation [GO:0033601] (biological process) Relationships: is a type of regulation of mammary gland epithelial cell proliferation [GO:0033599]; is a type of positive regulation of epithelial cell proliferation [GO:0050679]; is a type of positive regulation of developmental process [GO:0051094]; is a type of positive regulation of multicellular organismal process [GO:0051240]; positively regulates mammary gland epithelial cell proliferation [GO:0033598] Also known as: up regulation of mammary gland epithelial cell proliferation, up-regulation of mammary gland epithelial cell proliferation, upregulation of mammary gland epithelial cell proliferation, activation of mammary gland epithelial cell proliferation, stimulation of mammary gland epithelial cell proliferation Definition: Any process that activates or increases the rate or extent of mammary gland epithelial cell proliferation. Sources: GOC:mah